{
  "term_id": "UNKNOWN:0003",
  "gene_symbol": "C16orf54",
  "term_label": "Unknown cellular component",
  "gene": "UniProtKB:Q6UWD8",
  "gene_name": "Transmembrane protein C16orf54"
}